{
  "gene_symbol": "ADCY4",
  "term_id": "GO:0007189",
  "gene_name": "Adenylate cyclase type 4",
  "term_label": "adenylate cyclase-activating G protein-coupled receptor signaling pathway",
  "gene": "UniProtKB:Q8NFM4"
}